{
  "gene": "UniProtKB:Q6PIV7",
  "gene_symbol": "SLC25A34",
  "gene_name": "Solute carrier family 25 member 34",
  "term_label": "Unknown molecular function",
  "term_id": "UNKNOWN:0001"
}